L-phenylalanine catabolic process [GO:0006559] (biological process) Also known as: phenylalanine catabolic process, phenylalanine catabolism, L-phenylalanine breakdown, L-phenylalanine catabolism, L-phenylalanine degradation Sources: GOC:go_curators Relationships: is a type of L-phenylalanine metabolic process [GO:0006558]; is a type of GO:0009074; is_a L-amino acid catabolic process [GO:0170035]; is a type of GO:0170040 Definition: The chemical reactions and pathways resulting in the breakdown of L-phenylalanine, 2-amino-3-phenylpropanoic acid. Subtypes: anaerobic L-phenylalanine oxidation [GO:0019561]